negative regulation of fibroblast proliferation [GO:0048147] (biological process) Definition: Any process that stops, prevents, or reduces the frequency, rate or extent of multiplication or reproduction of fibroblast cells. Subtypes: negative regulation of hepatic stellate cell proliferation [GO:1904898], negative regulation of pancreatic stellate cell proliferation [GO:2000230] Relationships: is_a negative regulation of cell population proliferation [GO:0008285]; is a type of regulation of fibroblast proliferation [GO:0048145]; negatively regulates fibroblast proliferation [GO:0048144] Also known as: down regulation of fibroblast proliferation, down-regulation of fibroblast proliferation, downregulation of fibroblast proliferation, inhibition of fibroblast proliferation Sources: GOC:jid